{
  "gene": "UniProtKB:Q93045",
  "term_label": "cytoplasm",
  "gene_symbol": "STMN2",
  "gene_name": "Stathmin-2",
  "term_id": "GO:0005737"
}